alpha,alpha-trehalose phosphorylase activity [GO:0047656] (molecular function) Definition: Catalysis of the reaction: alpha,alpha-trehalose + phosphate = D-glucose + beta-D-glucose 1-phosphate. Relationships: is a type of 1,4-alpha-oligoglucan phosphorylase activity [GO:0004645] Sources: EC:2.4.1.64, MetaCyc:ALPHAALPHA-TREHALOSE-PHOSPHORYLASE-RXN Also known as: trehalose phosphorylase, a,a-trehalose phosphorylase activity, alpha,alpha-trehalose:phosphate beta-D-glucosyltransferase activity